{
  "gene": "UniProtKB:Q14696",
  "term_label": "Unknown cellular component",
  "gene_name": "LRP chaperone MESD",
  "gene_symbol": "MESD",
  "term_id": "UNKNOWN:0003"
}